atrial ventricular junction remodeling [GO:0003294] (biological process) Relationships: is a type of GO:0048771; is part of GO:0003007 Also known as: atrial ventricular junction remodelling, atrioventricular junction remodeling, atrio-ventricular junction remodeling Sources: GOC:mtg_heart Definition: The reorganization or renovation of heart tissue that contributes to the maturation of the connection between an atrium and a ventricle.